{
  "term_id": "GO:0035024",
  "gene_name": "Ras-interacting protein 1",
  "term_label": "negative regulation of Rho protein signal transduction",
  "gene_symbol": "RASIP1",
  "gene": "UniProtKB:Q5U651"
}